taxifolin 8-monooxygenase activity [GO:0050326] (molecular function) Sources: EC:1.14.13.19, MetaCyc:TAXIFOLIN-8-MONOOXYGENASE-RXN Relationships: is a type of oxidoreductase activity, acting on paired donors, with incorporation or reduction of molecular oxygen, NAD(P)H as one donor, and incorporation of one atom of oxygen [GO:0016709] Definition: Catalysis of the reaction: taxifolin + NAD(P)H + H+ + O2 = 2,3-dihydrogossypetin + NAD(P)+ + H2O. Also known as: taxifolin hydroxylase activity, taxifolin,NAD(P)H:oxygen oxidoreductase (8-hydroxylating)